regulation of translation by machinery localization [GO:0043143] (biological process) Relationships: is a type of regulation of translation [GO:0006417]; is a type of intracellular protein localization [GO:0008104]; BFO_0000050 translation [GO:0006412] Definition: Any process in which proteins and protein complexes involved in translation are transported to, or maintained in, a specific location. Sources: GOC:jl Also known as: establishment and maintenance of translational machinery localization, establishment and maintenance of translational protein localization, regulation of translation by machinery localisation, translational machinery localization, translational protein localization